{
  "gene": "UniProtKB:P40145",
  "gene_name": "Adenylate cyclase type 8",
  "gene_symbol": "ADCY8",
  "term_id": "GO:0007189",
  "term_label": "adenylate cyclase-activating G protein-coupled receptor signaling pathway"
}